{
  "gene": "UniProtKB:P35790",
  "gene_name": "Choline kinase alpha",
  "term_id": "GO:0006657",
  "gene_symbol": "CHKA",
  "term_label": "CDP-choline pathway"
}